{
  "gene_symbol": "SNRPD1",
  "gene": "UniProtKB:P62314",
  "gene_name": "Small nuclear ribonucleoprotein Sm D1",
  "term_id": "GO:0034719",
  "term_label": "SMN-Sm protein complex"
}